serine-tRNA ligase complex [GO:0140715] (cellular component) Relationships: is a type of catalytic complex [GO:1902494] Definition: A heterodimeric enzyme complex that catalyzes the ligation of serine to tRNA(Ser), forming L-seryl-tRNA(Ser). References: PMID:30943413